{
  "gene": "UniProtKB:Q96JW4",
  "gene_symbol": "SLC41A2",
  "term_id": "GO:0005886",
  "gene_name": "Solute carrier family 41 member 2",
  "term_label": "plasma membrane"
}